{
  "gene_name": "N-acetylneuraminate lyase",
  "gene": "UniProtKB:Q9BXD5",
  "gene_symbol": "NPL",
  "term_id": "UNKNOWN:0003",
  "term_label": "Unknown cellular component"
}